{
  "term_id": "GO:0051661",
  "gene": "UniProtKB:Q5T280",
  "gene_name": "Putative methyltransferase C9orf114",
  "term_label": "maintenance of centrosome location",
  "gene_symbol": "SPOUT1"
}